{
  "term_id": "UNKNOWN:0002",
  "gene": "UniProtKB:Q9H9V4",
  "gene_symbol": "RNF122",
  "gene_name": "RING finger protein 122",
  "term_label": "Unknown biological process"
}